{
  "term_label": "Unknown biological process",
  "gene_name": "Ubiquitin carboxyl-terminal hydrolase 2",
  "gene_symbol": "USP2",
  "term_id": "UNKNOWN:0002",
  "gene": "UniProtKB:O75604"
}